{
  "gene_symbol": "GCC1",
  "gene": "UniProtKB:Q96CN9",
  "gene_name": "GRIP and coiled-coil domain-containing protein 1",
  "term_id": "UNKNOWN:0002",
  "term_label": "Unknown biological process"
}